{
  "gene_symbol": "ATG2B",
  "gene_name": "Autophagy-related protein 2 homolog B",
  "gene": "UniProtKB:Q96BY7",
  "term_id": "GO:0034727",
  "term_label": "piecemeal microautophagy of the nucleus"
}